{
  "term_label": "regulation of transcription by RNA polymerase II",
  "term_id": "GO:0006357",
  "gene_name": "Forkhead box protein L2",
  "gene_symbol": "FOXL2",
  "gene": "UniProtKB:P58012"
}